{
  "term_label": "transmembrane receptor protein tyrosine kinase activity",
  "term_id": "GO:0004714",
  "gene_symbol": "NTRK3",
  "gene": "UniProtKB:Q16288",
  "gene_name": "NT-3 growth factor receptor"
}